positive regulation of endothelial cell-matrix adhesion [GO:1904906] (biological process) Also known as: up regulation of endothelial cell-matrix adhesion, up-regulation of endothelial cell-matrix adhesion, upregulation of endothelial cell-matrix adhesion, activation of endothelial cell-matrix adhesion Relationships: is a type of GO:0001954; is a type of regulation of endothelial cell-matrix adhesion [GO:1904904]; positively regulates endothelial cell-matrix adhesion [GO:0090673] Definition: Any process that activates or increases the frequency, rate or extent of endothelial cell-matrix adhesion. References: PMID:19460962 Sources: GOC:BHF, GOC:BHF_miRNA, GOC:TermGenie, GOC:bc, GO_REF:0000058